virus tail [GO:0098015] (cellular component) Also known as: bacteriophage tail, viral tail Note: Many bacteriophages with dsDNA genomes, or Caudovirales, have a tail. The viral tail can be short (Podoviridae), long and non-contractile (Siphoviridae) or long and contractile (Myoviridae). The tail is the channel through which the phage genome is injected into the host bacterial cell. Sources: GOC:bm, VZ:3958 Definition: Part of the virion that may be used to recognize, attach and inject the viral genome and accessory proteins into the host cell. Relationships: is a type of virion component [GO:0044423]